{
  "gene_symbol": "NOM1",
  "term_label": "nucleolus",
  "gene_name": "Nucleolar MIF4G domain-containing protein 1",
  "term_id": "GO:0005730",
  "gene": "UniProtKB:Q5C9Z4"
}